chromosomal region [GO:0098687] (cellular component) Subtypes: chromosome, centromeric region [GO:0000775], chromosome, telomeric region [GO:0000781], polytene chromosome puff [GO:0005703], polytene chromosome band [GO:0005704], GO:0005705, chromosome, centromeric core domain [GO:0034506] Note: Chromosomal regions include parts that are not part of the chromatin. Examples include the kinetochore. Also known as: chromosome region Sources: GOC:dos Relationships: is a type of cellular anatomical structure [GO:0110165]; is part of chromosome [GO:0005694] Definition: Any subdivision of a chromosome along its length.